{
  "gene_name": "Putative heat shock protein HSP 90-beta 4",
  "gene_symbol": "HSP90AB4P",
  "term_id": "GO:0050821",
  "term_label": "protein stabilization",
  "gene": "UniProtKB:Q58FF6"
}